{
  "term_label": "male meiosis chromosome separation",
  "gene": "UniProtKB:Q8TC57",
  "gene_symbol": "M1AP",
  "gene_name": "Meiosis 1 arrest protein",
  "term_id": "GO:0051308"
}